{
  "term_id": "UNKNOWN:0002",
  "term_label": "Unknown biological process",
  "gene_symbol": "ASPHD1",
  "gene": "UniProtKB:Q5U4P2",
  "gene_name": "Aspartate beta-hydroxylase domain-containing protein 1"
}